{
  "gene_symbol": "CSN1S1",
  "term_label": "response to dehydroepiandrosterone",
  "gene_name": "Alpha-S1-casein",
  "gene": "UniProtKB:P47710",
  "term_id": "GO:1903494"
}